{
  "gene_symbol": "MAP4K2",
  "term_label": "MAP kinase kinase kinase kinase activity",
  "gene": "UniProtKB:Q12851",
  "gene_name": "Mitogen-activated protein kinase kinase kinase kinase 2",
  "term_id": "GO:0008349"
}